regulation of muscle filament sliding speed involved in regulation of the velocity of shortening in skeletal muscle contraction [GO:0014915] (BP) Relationships: is a type of regulation of muscle filament sliding involved in regulation of the velocity of shortening in skeletal muscle contraction [GO:0014880]; is a type of GO:0032972 Sources: GOC:dph, GOC:mtg_muscle, GOC:tb Definition: Any process that modulates the velocity of muscle filament sliding, and consequently contributes to the regulation of the velocity of shortening of skeletal muscle contraction.